{
  "term_label": "Unknown molecular function",
  "gene_name": "Elongin-A",
  "gene_symbol": "ELOA",
  "term_id": "UNKNOWN:0001",
  "gene": "UniProtKB:Q14241"
}